regulation of sexual sporulation resulting in formation of a cellular spore [GO:0043940] (biological process) Relationships: is a type of GO:0034306; is a type of regulation of sporulation resulting in formation of a cellular spore [GO:0042173]; regulates GO:0043935 Definition: Any process that modulates the frequency, rate or extent of the formation of cellular spores derived from the products of meiosis. Sources: GOC:pamgo_curators Subtypes: regulation of ascospore formation [GO:0034307], positive regulation of sexual sporulation resulting in formation of a cellular spore [GO:0043941], GO:0043942, GO:0075244, regulation of zygospore formation [GO:0075298], GO:0075302